{
  "gene_name": "Aquaporin-7B",
  "gene": "UniProtKB:A0A075B734",
  "gene_symbol": "AQP7B",
  "term_id": "GO:0006833",
  "term_label": "water transport"
}